import into cell [GO:0098657] (BP) Also known as: uptake Subtypes: neurotransmitter uptake [GO:0001504], endocytosis [GO:0006897], GO:0009290, siderophore-iron import into cell [GO:0033214], long-chain fatty acid import into cell [GO:0044539], GO:0071939, GO:0098739 Definition: The directed movement of some substance from outside of a cell into a cell. This may occur via transport across the plasma membrane or via endocytosis. Sources: GOC:dos Relationships: is a type of transport [GO:0006810]